negative regulation of muscle cell apoptotic process [GO:0010656] (BP) Subtypes: negative regulation of striated muscle cell apoptotic process [GO:0010664], negative regulation of smooth muscle cell apoptotic process [GO:0034392] Also known as: negative regulation of muscle cell apoptosis Sources: GOC:dph, GOC:mtg_apoptosis, GOC:tb Definition: Any process that decreases the rate or frequency of muscle cell apoptotic process, a form of programmed cell death induced by external or internal signals that trigger the activity of proteolytic caspases whose actions dismantle a muscle cell and result in its death. Relationships: is a type of regulation of muscle cell apoptotic process [GO:0010660]; is a type of negative regulation of apoptotic process [GO:0043066]; negatively regulates GO:0010657